{
  "gene_symbol": "NR2E1",
  "gene_name": "Nuclear receptor subfamily 2 group E member 1",
  "term_id": "UNKNOWN:0003",
  "term_label": "Unknown cellular component",
  "gene": "UniProtKB:Q9Y466"
}